{
  "term_label": "detection of mechanical stimulus involved in sensory perception of sound",
  "gene_symbol": "TMC1",
  "gene_name": "Transmembrane channel-like protein 1",
  "term_id": "GO:0050910",
  "gene": "UniProtKB:Q8TDI8"
}